{
  "term_id": "GO:0071346",
  "gene_symbol": "GBP7",
  "gene": "UniProtKB:Q8N8V2",
  "gene_name": "Guanylate-binding protein 7",
  "term_label": "cellular response to type II interferon"
}